{
  "gene_name": "Histone H2B type 2-E",
  "term_id": "GO:0005615",
  "gene": "UniProtKB:Q16778",
  "term_label": "extracellular space",
  "gene_symbol": "H2BC21"
}